{
  "term_label": "cytoplasm",
  "gene_name": "Proteasome activator complex subunit 2",
  "gene": "UniProtKB:Q9UL46",
  "gene_symbol": "PSME2",
  "term_id": "GO:0005737"
}